{
  "term_label": "RNA binding",
  "gene": "UniProtKB:Q8IWA0",
  "gene_symbol": "WDR75",
  "term_id": "GO:0003723",
  "gene_name": "WD repeat-containing protein 75"
}